{
  "term_id": "UNKNOWN:0002",
  "gene_name": "Heterogeneous nuclear ribonucleoprotein C-like 1",
  "gene_symbol": "HNRNPCL1",
  "term_label": "Unknown biological process",
  "gene": "UniProtKB:O60812"
}